phosphoenolpyruvate carboxykinase (diphosphate) activity [GO:0030585] (molecular function) Relationships: is a type of phosphoenolpyruvate carboxykinase activity [GO:0004611] Also known as: phosphoenolpyruvic carboxykinase, phosphopyruvate carboxykinase, PEP carboxyphosphotransferase activity, PEPCTrP, diphosphate:oxaloacetate carboxy-lyase (transphosphorylating), diphosphate:oxaloacetate carboxy-lyase (transphosphorylating; phosphoenolpyruvate-forming), phosphoenolpyruvate carboxykinase (pyrophosphate) activity, phosphoenolpyruvate carboxylase (pyrophosphate), phosphoenolpyruvate carboxyphosphotransferase activity, phosphoenolpyruvate carboxytransphosphorylase activity, phosphoenolpyruvic carboxykinase (pyrophosphate), phosphoenolpyruvic carboxylase (pyrophosphate), phosphoenolpyruvic carboxytransphosphorylase activity, phosphopyruvate carboxykinase (pyrophosphate), phosphopyruvate carboxylase (pyrophosphate) Sources: EC:4.1.1.38, RHEA:22356 Definition: Catalysis of the reaction: diphosphate + oxaloacetate = CO2 + phosphate + phosphoenolpyruvate.